{
  "term_id": "UNKNOWN:0001",
  "term_label": "Unknown molecular function",
  "gene": "UniProtKB:A0A075B6P5",
  "gene_name": "Immunoglobulin kappa variable 2-28",
  "gene_symbol": "IGKV2-28"
}